{
  "term_label": "mitochondrion",
  "gene_name": "Isoleucine--tRNA ligase, mitochondrial",
  "gene_symbol": "IARS2",
  "term_id": "GO:0005739",
  "gene": "UniProtKB:Q9NSE4"
}